{
  "term_id": "GO:0006900",
  "gene": "UniProtKB:Q9NZZ3",
  "gene_name": "Charged multivesicular body protein 5",
  "term_label": "vesicle budding from membrane",
  "gene_symbol": "CHMP5"
}